{
  "term_id": "GO:0006110",
  "gene": "UniProtKB:Q9UGI9",
  "gene_name": "5'-AMP-activated protein kinase subunit gamma-3",
  "gene_symbol": "PRKAG3",
  "term_label": "regulation of glycolytic process"
}